viridicatumtoxin biosynthetic process [GO:0140872] (biological process) References: PMID:20534346, PMID:24161266 Definition: The chemical reactions and pathways resulting in the formation of viridicatumtoxin, a tetracycline-like fungal meroterpenoid with a unique, fused spirobicyclic ring system. Also known as: viridicatumtoxin anabolism, viridicatumtoxin biosynthesis, viridicatumtoxin formation, viridicatumtoxin synthesis Relationships: is a type of polyketide biosynthetic process [GO:0030639]; is a type of ketone biosynthetic process [GO:0042181]; is a type of mycotoxin biosynthetic process [GO:0043386]; is_a amide biosynthetic process [GO:0043604]; is a type of GO:0046189; is a type of olefinic compound biosynthetic process [GO:0120255]; is a type of GO:1901503; is a type of tertiary alcohol biosynthetic process [GO:1902645]; is a type of secondary alcohol biosynthetic process [GO:1902653]